positive regulation of mini excitatory postsynaptic potential [GO:0061885] (biological process) Definition: Any process that increases the frequency, rate or extent of mini excitatory postsynaptic potential. Mini excitatory postsynaptic potential is a process that leads to a temporary increase in postsynaptic potential due to the flow of positively charged ions into the postsynaptic cell, induced by the spontaneous release of a single vesicle of an excitatory neurotransmitter into the synapse. References: PMID:20395454 Sources: GOC:aruk, GOC:bc Relationships: is a type of regulation of mini excitatory postsynaptic potential [GO:0061884]; is a type of positive regulation of excitatory postsynaptic potential [GO:2000463]; positively regulates GO:0098816